{
  "gene_symbol": "HMCES",
  "term_label": "replication fork",
  "gene_name": "Abasic site processing protein HMCES",
  "gene": "UniProtKB:Q96FZ2",
  "term_id": "GO:0005657"
}